negative regulation of protein targeting to membrane [GO:0090315] (biological process) Relationships: is a type of negative regulation of cellular process [GO:0048523]; is a type of regulation of protein targeting to membrane [GO:0090313]; is_a negative regulation of establishment of protein localization [GO:1904950]; negatively regulates protein targeting to membrane [GO:0006612] Sources: GOC:tb Subtypes: negative regulation of protein targeting to vacuolar membrane [GO:1900484] Definition: Any process that decreases the frequency, rate or extent of the process of directing proteins towards a membrane, usually using signals contained within the protein.